{
  "gene_name": "Nuclear pore complex-interacting protein family member B4",
  "gene": "UniProtKB:C9JG80",
  "term_id": "UNKNOWN:0001",
  "gene_symbol": "NPIPB4",
  "term_label": "Unknown molecular function"
}